{
  "gene_symbol": "DMBX1",
  "term_id": "UNKNOWN:0003",
  "gene_name": "Diencephalon_mesencephalon homeobox protein 1",
  "gene": "UniProtKB:Q8NFW5",
  "term_label": "Unknown cellular component"
}